L-alanine catabolic process, by transamination [GO:0019481] (biological process) Also known as: L-alanine breakdown, by transamination, L-alanine degradation, by transamination Relationships: is a type of L-alanine catabolic process [GO:0042853] Definition: The chemical reactions and pathways resulting in the breakdown of L-alanine by transamination. Sources: GOC:go_curators